{
  "gene_name": "Gamma-tubulin complex component 5",
  "term_id": "GO:0007020",
  "gene_symbol": "TUBGCP5",
  "term_label": "microtubule nucleation",
  "gene": "UniProtKB:Q96RT8"
}